regulation of sodium ion import across plasma membrane [GO:1903782] (biological process) Subtypes: negative regulation of sodium ion import across plasma membrane [GO:1903783], positive regulation of sodium ion import across plasma membrane [GO:1903784] References: PMID:19376779 Sources: GOC:BHF, GOC:TermGenie, GOC:mtg_cardiac_conduct_nov11, GOC:nc, GO_REF:0000058 Definition: Any process that modulates the frequency, rate or extent of sodium ion import across the plasma membrane. Relationships: is a type of GO:1902305; regulates sodium ion import across plasma membrane [GO:0098719]